MDA-5 binding [GO:0039556] (molecular function) Definition: Binding to MDA-5, a cytoplasmic pattern recognition receptor that initiates an antiviral signaling pathway upon binding to viral dsRNA. References: PMID:19019954 Relationships: is a type of signaling receptor binding [GO:0005102] Also known as: MDA5 binding